follicle-stimulating hormone secretion [GO:0046884] (biological process) Definition: The regulated release of follicle-stimulating hormone, a gonadotropic glycoprotein hormone secreted by the anterior pituitary. Also known as: FSH secretion, follicle stimulating hormone secretion, follitropin secretion Regulation: regulated by regulation of follicle-stimulating hormone secretion [GO:0046880]; positively regulated by GO:0046881; negatively regulated by negative regulation of follicle-stimulating hormone secretion [GO:0046882] Sources: ISBN:0198506732 Relationships: is a type of gonadotropin secretion [GO:0032274]